{
  "gene_symbol": "TLE5",
  "term_label": "Unknown cellular component",
  "term_id": "UNKNOWN:0003",
  "gene_name": "TLE family member 5",
  "gene": "UniProtKB:Q08117"
}